response to candesartan [GO:1901556] (BP) Definition: Any process that results in a change in state or activity of a cell or an organism (in terms of movement, secretion, enzyme production, gene expression, etc.) as a result of a candesartan stimulus. Relationships: is a type of GO:1901698; is a type of response to oxygen-containing compound [GO:1901700] Sources: GOC:TermGenie